{
  "gene_name": "Galectin-3",
  "gene": "UniProtKB:P17931",
  "gene_symbol": "LGALS3",
  "term_id": "GO:0048246",
  "term_label": "macrophage chemotaxis"
}